tRNA processing [GO:0008033] (biological process) Also known as: tRNA maturation Regulation: RO_0002211 by GO:2000235; negatively regulated by negative regulation of tRNA processing [GO:2000236]; positively regulated by GO:2000237 Definition: The process in which a pre-tRNA molecule is converted to a mature tRNA, ready for addition of an aminoacyl group. Subtypes: GO:0006388, GO:0006400, tRNA 3'-end processing [GO:0042780], GO:0090646, tRNA 5'-end processing [GO:0099116] References: PMID:12533506 Sources: GOC:jl Relationships: is a type of RNA processing [GO:0006396]; is a type of tRNA metabolic process [GO:0006399]